{
  "gene": "UniProtKB:Q9NQX4",
  "term_id": "GO:0000146",
  "gene_symbol": "MYO5C",
  "term_label": "microfilament motor activity",
  "gene_name": "Unconventional myosin-Vc"
}